{
  "gene_name": "Mucin-6",
  "gene_symbol": "MUC6",
  "term_id": "UNKNOWN:0002",
  "gene": "UniProtKB:Q6W4X9",
  "term_label": "Unknown biological process"
}